positive regulation of nucleoside transport [GO:0032244] (biological process) Relationships: is a type of GO:0032241; is_a GO:0032242; positively regulates nucleoside transport [GO:0015858] Sources: GOC:mah Subtypes: positive regulation of purine nucleoside transport [GO:0032248] Definition: Any process that activates or increases the frequency, rate or extent of the directed movement of a nucleoside into, out of or within a cell, or between cells, by means of some agent such as a transporter or pore. Also known as: up regulation of nucleoside transport, up-regulation of nucleoside transport, upregulation of nucleoside transport, activation of nucleoside transport, stimulation of nucleoside transport